{
  "gene": "UniProtKB:Q96EQ0",
  "term_id": "GO:0060090",
  "term_label": "molecular adaptor activity",
  "gene_symbol": "SGTB",
  "gene_name": "Small glutamine-rich tetratricopeptide repeat-containing protein beta"
}